{
  "term_id": "GO:0004089",
  "gene_symbol": "CA7",
  "gene_name": "Carbonic anhydrase 7",
  "term_label": "carbonate dehydratase activity",
  "gene": "UniProtKB:P43166"
}